positive regulation of platelet-derived growth factor receptor signaling pathway [GO:0010641] (biological process) Definition: Any process that increases the frequency, rate or extent of the platelet-derived growth factor receptor signaling pathway. Relationships: is a type of GO:0009967; is a type of regulation of platelet-derived growth factor receptor signaling pathway [GO:0010640]; positively regulates GO:0048008 Subtypes: positive regulation of platelet-derived growth factor receptor-alpha signaling pathway [GO:2000585], positive regulation of platelet-derived growth factor receptor-beta signaling pathway [GO:2000588] Sources: GOC:dph, GOC:hjd, GOC:tb Also known as: positive regulation of platelet-derived growth factor receptor signalling pathway